negative regulation of tolerance induction dependent upon immune response [GO:0002653] (BP) Definition: Any process that stops, prevents, or reduces the frequency, rate, or extent of tolerance induction dependent upon immune response. Sources: GOC:add Also known as: down regulation of tolerance induction dependent upon immune response, down-regulation of tolerance induction dependent upon immune response, downregulation of tolerance induction dependent upon immune response, negative regulation of immune response-dependent tolerance induction, inhibition of tolerance induction dependent upon immune response Relationships: is a type of negative regulation of tolerance induction [GO:0002644]; is a type of regulation of tolerance induction dependent upon immune response [GO:0002652]; is a type of negative regulation of adaptive immune response based on somatic recombination of immune receptors built from immunoglobulin superfamily domains [GO:0002823]; negatively regulates tolerance induction dependent upon immune response [GO:0002461] Subtypes: negative regulation of tolerance induction to nonself antigen [GO:0002656], negative regulation of peripheral tolerance induction [GO:0002659]